C-X-C chemokine receptor CXCR4 signaling pathway [GO:0038159] (biological process) Relationships: is a type of chemokine-mediated signaling pathway [GO:0070098] Sources: GOC:nhn, GOC:signaling Also known as: CXCR4 signaling pathway Subtypes: CXCL12-activated CXCR4 signaling pathway [GO:0038160] Definition: The series of molecular signals initiated by a the C-X-C chemokine type 4 receptor on the surface of a cell binding to one of it's physiological ligands, and ending with the regulation of a downstream cellular process, e.g. transcription.